{
  "gene": "UniProtKB:P10809",
  "gene_symbol": "HSPD1",
  "term_label": "mitochondrial inner membrane",
  "gene_name": "60 kDa heat shock protein, mitochondrial",
  "term_id": "GO:0005743"
}